formaldehyde biosynthetic process [GO:0046293] (biological process) Also known as: formaldehyde anabolism, formaldehyde biosynthesis, formaldehyde formation, formaldehyde synthesis, methanal biosynthesis, methanal biosynthetic process Sources: GOC:ai Relationships: is a type of small molecule biosynthetic process [GO:0044283]; is a type of aldehyde biosynthetic process [GO:0046184]; is a type of formaldehyde metabolic process [GO:0046292] Definition: The chemical reactions and pathways resulting in the formation of formaldehyde (methanal, H2C=O), the simplest aldehyde.